{
  "gene": "UniProtKB:C9JG80",
  "term_label": "Unknown cellular component",
  "term_id": "UNKNOWN:0003",
  "gene_name": "Nuclear pore complex-interacting protein family member B4",
  "gene_symbol": "NPIPB4"
}